emericellin biosynthetic process [GO:1900766] (biological process) Also known as: emericellin anabolism, emericellin biosynthesis, emericellin formation, emericellin synthesis, Variecoxanthone B anabolism, Variecoxanthone B biosynthesis, Variecoxanthone B biosynthetic process, Variecoxanthone B formation, Variecoxanthone B synthesis Definition: The chemical reactions and pathways resulting in the formation of emericellin. Regulation: regulated by GO:1900834; negatively regulated by GO:1900835; positively regulated by positive regulation of emericellin biosynthetic process [GO:1900836] Relationships: is_a secondary metabolite biosynthetic process [GO:0044550]; is a type of phenol-containing compound biosynthetic process [GO:0046189]; is a type of ether biosynthetic process [GO:1901503]; is a type of xanthone-containing compound biosynthetic process [GO:2001307] Sources: GOC:TermGenie, GOC:di